meiotic heteroduplex formation [GO:0000713] (biological process) References: PMID:9334324 Sources: GOC:elh Relationships: is a type of meiosis I cell cycle process [GO:0061982]; is part of DNA recombination [GO:0006310] Definition: During meiosis, the formation of a stable duplex DNA that contains one strand from each of the two recombining DNA molecules.